{
  "gene": "UniProtKB:Q15276",
  "term_id": "GO:0030139",
  "term_label": "endocytic vesicle",
  "gene_name": "Rab GTPase-binding effector protein 1",
  "gene_symbol": "RABEP1"
}